{
  "term_id": "GO:0031430",
  "term_label": "M band",
  "gene_name": "Titin",
  "gene": "UniProtKB:Q8WZ42",
  "gene_symbol": "TTN"
}